{
  "gene_name": "Chromodomain-helicase-DNA-binding protein 5",
  "gene": "UniProtKB:Q8TDI0",
  "term_label": "chromatin binding",
  "term_id": "GO:0003682",
  "gene_symbol": "CHD5"
}